{
  "gene_symbol": "ERH",
  "term_id": "UNKNOWN:0003",
  "gene": "UniProtKB:P84090",
  "term_label": "Unknown cellular component",
  "gene_name": "Enhancer of rudimentary homolog"
}